cellular response to chondroitin 6'-sulfate [GO:1905440] (BP) References: PMID:22365850 Sources: GOC:TermGenie, GO_REF:0000071 Relationships: is a type of GO:1901699; is a type of cellular response to oxygen-containing compound [GO:1901701]; is a type of response to chondroitin 6'-sulfate [GO:1905439] Definition: Any process that results in a change in state or activity of a cell (in terms of movement, secretion, enzyme production, gene expression, etc.) as a result of a chondroitin 6'-sulfate stimulus.